{
  "gene": "UniProtKB:Q9BSW2",
  "term_id": "GO:0016192",
  "term_label": "vesicle-mediated transport",
  "gene_name": "EF-hand calcium-binding domain-containing protein 4B",
  "gene_symbol": "CRACR2A"
}